{
  "term_id": "GO:0086080",
  "gene_name": "Izumo sperm-egg fusion protein 1",
  "gene": "UniProtKB:Q8IYV9",
  "gene_symbol": "IZUMO1",
  "term_label": "protein binding involved in heterotypic cell-cell adhesion"
}